{
  "term_label": "ferrous iron binding",
  "gene_name": "Ferritin light chain",
  "gene": "UniProtKB:P02792",
  "gene_symbol": "FTL",
  "term_id": "GO:0008198"
}